positive regulation of penetration peg formation [GO:0075055] (biological process) Definition: Any process that activates, maintains or increases the frequency, rate or extent of symbiont penetration peg formation for entry into host. The host is defined as the larger of the organisms involved in a symbiotic interaction. Also known as: positive regulation of symbiont penetration peg formation for entry into host, positive regulation of symbiont penetration peg initiation Note: Note that this term should not be used to annotate gene products of the host. It should only be used to annotate those gene products from the symbiont involved in this process. Relationships: is a type of positive regulation of developmental process [GO:0051094]; is a type of modulation of penetration peg formation [GO:0075054]; is a type of positive regulation by symbiont of entry into host [GO:0075294]; positively regulates GO:0075053 Sources: GOC:pamgo_curators